{
  "gene_name": "G antigen 10",
  "term_id": "UNKNOWN:0001",
  "gene_symbol": "GAGE10",
  "gene": "UniProtKB:A6NGK3",
  "term_label": "Unknown molecular function"
}